regulation of blood vessel endothelial cell proliferation involved in sprouting angiogenesis [GO:1903587] (biological process) References: PMID:23388056 Sources: GOC:TermGenie, GO_REF:0000058 Relationships: is a type of regulation of endothelial cell proliferation [GO:0001936]; regulates blood vessel endothelial cell proliferation involved in sprouting angiogenesis [GO:0002043] Also known as: regulation of blood vessel endothelial cell proliferation during sprouting angiogenesis Subtypes: negative regulation of blood vessel endothelial cell proliferation involved in sprouting angiogenesis [GO:1903588], GO:1903589 Definition: Any process that modulates the frequency, rate or extent of blood vessel endothelial cell proliferation involved in sprouting angiogenesis.